actin cortical patch localization [GO:0051666] (biological process) Sources: GOC:mah Relationships: is a type of cellular localization [GO:0051641] Also known as: actin cortical patch localisation, establishment and maintenance of actin cortical patch localization Definition: Any process in which actin cortical patches are transported to, or maintained in, a specific location. An actin cortical patch is a discrete actin-containing structure found just beneath the plasma membrane in fungal cells. Regulation: regulated by regulation of actin cortical patch localization [GO:0060583]